{
  "gene_name": "Uncharacterized protein encoded by LINC01600",
  "term_id": "UNKNOWN:0003",
  "gene": "UniProtKB:Q96MT4",
  "gene_symbol": "LINC01600",
  "term_label": "Unknown cellular component"
}